{
  "term_label": "Unknown molecular function",
  "gene": "UniProtKB:A0A0B4J235",
  "gene_name": "T cell receptor alpha variable 13-2",
  "gene_symbol": "TRAV13-2",
  "term_id": "UNKNOWN:0001"
}